{
  "gene": "UniProtKB:Q6ZVT0",
  "term_label": "Unknown biological process",
  "gene_symbol": "TTLL10",
  "gene_name": "Inactive polyglycylase TTLL10",
  "term_id": "UNKNOWN:0002"
}